{
  "gene": "UniProtKB:Q9UK45",
  "term_id": "GO:0097526",
  "gene_name": "U6 snRNA-associated Sm-like protein LSm7",
  "gene_symbol": "LSM7",
  "term_label": "spliceosomal tri-snRNP complex"
}